{
  "gene": "UniProtKB:Q9H0R5",
  "gene_symbol": "GBP3",
  "gene_name": "Guanylate-binding protein 3",
  "term_id": "GO:0071346",
  "term_label": "cellular response to type II interferon"
}